{
  "term_id": "GO:0007165",
  "gene": "UniProtKB:O00468",
  "term_label": "signal transduction",
  "gene_name": "Agrin",
  "gene_symbol": "AGRN"
}